{
  "gene_symbol": "SKAP2",
  "gene_name": "Src kinase-associated phosphoprotein 2",
  "term_id": "GO:0005737",
  "term_label": "cytoplasm",
  "gene": "UniProtKB:O75563"
}